gastrulation with mouth forming first [GO:0001703] (biological process) Definition: A gastrulation process in which the initial invagination becomes the mouth and the anus forms second. Subtypes: gastrulation involving germ band extension [GO:0010004] Relationships: is_a gastrulation [GO:0007369] Also known as: protostomic gastrulation Sources: GOC:go_curators, GOC:mtg_sensu